{
  "gene": "UniProtKB:Q12988",
  "gene_symbol": "HSPB3",
  "term_label": "Unknown molecular function",
  "term_id": "UNKNOWN:0001",
  "gene_name": "Heat shock protein beta-3"
}